tRNA C5-cytosine methylation [GO:0002946] (biological process) Definition: The process whereby a cytosine in a tRNA is methylated at position 5 of the cytosine. Sources: ISBN:155581073X Relationships: is a type of GO:0030488 Subtypes: tRNA wobble base cytosine methylation [GO:0002127] Also known as: tRNA 5-methylcytosine biosynthesis Regulation: regulated by GO:0110003; positively regulated by positive regulation of tRNA C5-cytosine methylation [GO:0110005]